{
  "term_label": "cytoplasm",
  "gene_symbol": "HERC3",
  "gene": "UniProtKB:Q15034",
  "gene_name": "Probable E3 ubiquitin-protein ligase HERC3",
  "term_id": "GO:0005737"
}